{
  "gene": "UniProtKB:Q9P0K7",
  "term_label": "Unknown molecular function",
  "term_id": "UNKNOWN:0001",
  "gene_name": "Ankycorbin",
  "gene_symbol": "RAI14"
}